negative regulation of oocyte karyosome formation [GO:0120314] (BP) Definition: Any process that stops, prevents, or reduces the frequency, rate or extent of oocyte karyosome formation, the chromosome organization process in which meiotic chromosomes in the oocyte nucleus cluster together to form a compact spherical structure called the karyosome. Relationships: is a type of negative regulation of cell cycle process [GO:0010948]; is a type of regulation of oocyte karyosome formation [GO:0120313]; is a type of negative regulation of reproductive process [GO:2000242]; is a type of negative regulation of chromosome organization [GO:2001251]; negatively regulates oocyte karyosome formation [GO:0030717] References: PMID:33382409 Sources: GOC:ha, GOC:krc